3-phenylpropionate dioxygenase activity [GO:0008695] (molecular function) Definition: Catalysis of the reaction: 3-phenylpropionate + NADH + H+ + O2 = NAD+ + cis-3-(3-carboxyethyl)-3,5-cyclohexadiene-1,2-diol. Sources: UM-BBD_enzymeID:e0307 Also known as: 3-phenylpropanoate dioxygenase activity, 3-phenylpropanoate,NADH:oxygen oxidoreductase (2,3-hydroxylating) activity, Hca dioxygenase activity, HcaA1A2CD Relationships: is a type of oxidoreductase activity, acting on paired donors, with incorporation or reduction of molecular oxygen, NAD(P)H as one donor, and incorporation of two atoms of oxygen into one donor [GO:0016708]